{
  "term_label": "regulation of pyruvate decarboxylation to acetyl-CoA",
  "gene_symbol": "PDK1",
  "gene_name": "[Pyruvate dehydrogenase (acetyl-transferring)] kinase isozyme 1, mitochondrial",
  "gene": "UniProtKB:Q15118",
  "term_id": "GO:0010510"
}